{
  "gene_symbol": "RALGAPA1",
  "term_label": "Unknown biological process",
  "term_id": "UNKNOWN:0002",
  "gene_name": "Ral GTPase-activating protein subunit alpha-1",
  "gene": "UniProtKB:Q6GYQ0"
}